3-carboxy-cis,cis-muconate cycloisomerase activity [GO:0047472] (molecular function) Also known as: 3-carboxymuconate cycloisomerase type II activity, 3-carboxymuconate lactonizing enzyme activity, 3-carboxymuconolactone hydrolase activity, CMLE activity, beta-carboxymuconate lactonizing enzyme activity Definition: Catalysis of the reaction: 2-(carboxymethyl)-5-oxo-2,5-dihydro-2-furoate = 3-carboxy-cis,cis-muconate + H+. Relationships: is a type of intramolecular lyase activity [GO:0016872] References: PMID:15301541, PMID:17054713 Sources: RHEA:23656